{
  "term_label": "cell surface receptor signaling pathway",
  "gene_symbol": "ADGRA2",
  "gene_name": "Adhesion G protein-coupled receptor A2",
  "term_id": "GO:0007166",
  "gene": "UniProtKB:Q96PE1"
}